{
  "gene_name": "CapZ-interacting protein",
  "gene_symbol": "RCSD1",
  "term_id": "GO:0042147",
  "gene": "UniProtKB:Q6JBY9",
  "term_label": "retrograde transport, endosome to Golgi"
}